{
  "term_id": "UNKNOWN:0002",
  "gene": "UniProtKB:A0A286YF18",
  "gene_symbol": "SMIM44",
  "term_label": "Unknown biological process",
  "gene_name": "Small integral membrane protein 44"
}